{
  "term_id": "GO:0000245",
  "gene": "UniProtKB:P78362",
  "gene_name": "SRSF protein kinase 2",
  "gene_symbol": "SRPK2",
  "term_label": "spliceosomal complex assembly"
}